{
  "term_label": "synaptic vesicle membrane",
  "term_id": "GO:0030672",
  "gene": "UniProtKB:Q9P2U7",
  "gene_symbol": "SLC17A7",
  "gene_name": "Vesicular glutamate transporter 1"
}